{
  "term_id": "GO:0005688",
  "gene_name": "U6 snRNA-associated Sm-like protein LSm6",
  "term_label": "U6 snRNP",
  "gene": "UniProtKB:P62312",
  "gene_symbol": "LSM6"
}